G protein-coupled glutamate receptor binding [GO:0035256] (molecular function) Definition: Binding to a G protein-coupled glutamate receptor (a metabotropic glutamate receptor). References: PMID:9069287 Sources: GOC:bf, ISBN:0198506732 Also known as: G-protein coupled glutamate receptor binding, metabotropic glutamate receptor binding Relationships: is a type of G protein-coupled receptor binding [GO:0001664]; is a type of glutamate receptor binding [GO:0035254] Subtypes: type 1 metabotropic glutamate receptor binding [GO:0031798], type 2 metabotropic glutamate receptor binding [GO:0031799], type 3 metabotropic glutamate receptor binding [GO:0031800], type 4 metabotropic glutamate receptor binding [GO:0031801], type 5 metabotropic glutamate receptor binding [GO:0031802], type 6 metabotropic glutamate receptor binding [GO:0031803], GO:0031804, type 8 metabotropic glutamate receptor binding [GO:0031805]